{
  "gene_name": "Neuronal pentraxin-2",
  "gene": "UniProtKB:P47972",
  "term_id": "UNKNOWN:0002",
  "term_label": "Unknown biological process",
  "gene_symbol": "NPTX2"
}